{
  "gene": "UniProtKB:P05423",
  "term_id": "GO:0005666",
  "term_label": "RNA polymerase III complex",
  "gene_symbol": "POLR3D",
  "gene_name": "DNA-directed RNA polymerase III subunit RPC4"
}